{
  "term_label": "positive regulation of cell population proliferation",
  "gene_name": "Interleukin-12 receptor subunit beta-1",
  "gene_symbol": "IL12RB1",
  "term_id": "GO:0008284",
  "gene": "UniProtKB:P42701"
}